cellular response to arsenic-containing substance [GO:0071243] (biological process) Sources: GOC:mah Also known as: cellular response to arsenic Subtypes: cellular response to arsenite(3-) [GO:1903841], cellular response to arsenite ion [GO:1903843], GO:1903936 Definition: Any process that results in a change in state or activity of a cell (in terms of movement, secretion, enzyme production, gene expression, etc.) as a result of an arsenic stimulus from compounds containing arsenic, including arsenates, arsenites, and arsenides. Relationships: is a type of GO:0046685; is a type of cellular response to chemical stimulus [GO:0070887]